cytoplasmic side of trans-Golgi network membrane [GO:0160281] (cellular component) Definition: The leaflet of the membrane bilayer of the trans-Golgi network faces the cytoplasm and is crucial for lipid and protein sorting and trafficking, as it interacts with cytoplasmic proteins involved in vesicle formation and targeting. References: PMID:10922460, PMID:23913272, PMID:34597626 Relationships: is a type of cytoplasmic side of membrane [GO:0098562]; is part of trans-Golgi network membrane [GO:0032588] Also known as: cytoplasmic face of trans-Golgi network membrane, cytoplasmic leaflet of trans-Golgi network membrane, cytoplasmic side of trans-Golgi network